activated CD8-positive, alpha-beta T cell proliferation [GO:0035742] (biological process) Relationships: is a type of CD8-positive, alpha-beta T cell proliferation [GO:0035740] Sources: CL:0000906, GOC:BHF Definition: The expansion of an activated CD8-positive, alpha-beta T cell population by cell division.